cellular response to oxidised low-density lipoprotein particle stimulus [GO:0140052] (biological process) Definition: Any process that results in a change in state or activity of a cell (in terms of movement, secretion, enzyme production, gene expression, etc.) as a result of an oxidized lipoprotein particle stimulus. Also known as: cellular response to ox-LDL particle stimulus, cellular response to oxLDL particle stimulus, cellular response to oxidised LDL particle stimulus, cellular response to oxidized LDL particle stimulus, cellular response to oxidized low-density lipoprotein particle stimulus Relationships: is a type of GO:0071404 References: PMID:20037584, PMID:27607416 Sources: GOC:BHF, GOC:aruk